CD8-positive, alpha-beta T cell differentiation [GO:0043374] (biological process) Regulation: regulated by regulation of CD8-positive, alpha-beta T cell differentiation [GO:0043376]; negatively regulated by GO:0043377; positively regulated by positive regulation of CD8-positive, alpha-beta T cell differentiation [GO:0043378] Note: Note that immunologists typically use the word 'development' to refer to cells of B or T cell lineages undergoing the process that GO describes as 'cell differentiation'. Subtypes: CD8-positive, alpha-beta intraepithelial T cell differentiation [GO:0002300], CD8-positive, alpha-beta T cell differentiation involved in immune response [GO:0002302], CD8-positive, alpha-beta regulatory T cell differentiation [GO:0002307], CD8-positive, alpha-beta cytotoxic T cell differentiation [GO:0002308] Sources: ISBN:0781735149 Definition: The process in which a relatively unspecialized T cell acquires specialized features of a mature CD8-positive, alpha-beta T cell. Relationships: is a type of CD8-positive, alpha-beta T cell activation [GO:0036037]; is a type of alpha-beta T cell differentiation [GO:0046632] Also known as: CD8-positive, alpha-beta T lymphocyte differentiation, CD8-positive, alpha-beta T-cell differentiation, CD8-positive, alpha-beta T-lymphocyte differentiation, CD8-positive, alpha-beta T cell development